nucleologenesis [GO:0017126] (biological process) Definition: A cellular process that results in the biosynthesis of constituent macromolecules, assembly, and arrangement of constituent parts of a nucleolus, a small, dense body one or more of which are present in the nucleus of eukaryotic cells. Sources: GOC:jl, ISBN:0198506732 Also known as: nucleolus biogenesis, nucleolus assembly Relationships: is a type of nucleolus organization [GO:0007000]; is a type of cellular component biogenesis [GO:0044085]